{
  "gene": "UniProtKB:Q9HCE5",
  "gene_name": "N6-adenosine-methyltransferase non-catalytic subunit",
  "term_id": "GO:0036396",
  "gene_symbol": "METTL14",
  "term_label": "RNA N6-methyladenosine methyltransferase complex"
}